{
  "gene_symbol": "ICA1L",
  "term_label": "membrane curvature sensor activity",
  "gene_name": "Islet cell autoantigen 1-like protein",
  "term_id": "GO:0140090",
  "gene": "UniProtKB:Q8NDH6"
}